{
  "term_id": "GO:0030154",
  "gene": "UniProtKB:P78545",
  "gene_name": "ETS-related transcription factor Elf-3",
  "gene_symbol": "ELF3",
  "term_label": "cell differentiation"
}